{
  "term_id": "GO:0019814",
  "gene_name": "T cell receptor alpha variable 8-4",
  "term_label": "immunoglobulin complex",
  "gene": "UniProtKB:P01737",
  "gene_symbol": "TRAV8-4"
}